{
  "gene_symbol": "ZFP14",
  "term_id": "GO:0000978",
  "gene_name": "Zinc finger protein 14 homolog",
  "gene": "UniProtKB:Q9HCL3",
  "term_label": "RNA polymerase II cis-regulatory region sequence-specific DNA binding"
}